{
  "gene_symbol": "NLGN3",
  "term_id": "GO:0007158",
  "gene_name": "Neuroligin-3",
  "term_label": "neuron cell-cell adhesion",
  "gene": "UniProtKB:Q9NZ94"
}